{
  "gene": "UniProtKB:Q86T90",
  "gene_symbol": "KIAA1328",
  "term_label": "Unknown cellular component",
  "term_id": "UNKNOWN:0003",
  "gene_name": "Protein hinderin"
}